{
  "gene_name": "F-box only protein 4",
  "gene": "UniProtKB:Q9UKT5",
  "term_label": "SCF-dependent proteasomal ubiquitin-dependent protein catabolic process",
  "gene_symbol": "FBXO4",
  "term_id": "GO:0031146"
}